{
  "gene": "UniProtKB:Q8TDI7",
  "gene_name": "Transmembrane channel-like protein 2",
  "term_id": "UNKNOWN:0003",
  "term_label": "Unknown cellular component",
  "gene_symbol": "TMC2"
}